{
  "gene_symbol": "DIP2A",
  "term_label": "Unknown biological process",
  "gene": "UniProtKB:Q14689",
  "gene_name": "Disco-interacting protein 2 homolog A",
  "term_id": "UNKNOWN:0002"
}